STAT family protein binding [GO:0097677] (molecular function) References: PMID:21447371, PMID:24470978 Sources: GOC:mr, InterPro:IPR001217 Relationships: is a type of GO:0061629 Also known as: signal transducers and activators of transcription family protein binding Definition: Binding to a member of the signal transducers and activators of transcription (STAT) protein family. STATs are, as the name indicates, both signal transducers and transcription factors. STATs are activated by cytokines and some growth factors and thus control important biological processes including cell growth, cell differentiation, apoptosis and immune responses.